fatty acid beta-oxidation, unsaturated, even number, reductase/isomerase pathway [GO:0033543] (biological process) Relationships: is a type of fatty acid beta-oxidation, unsaturated, even number [GO:0033542] Definition: A fatty acid beta-oxidation pathway by which fatty acids having cis-double bonds on even-numbered carbons are degraded. In this pathway, the intermediate 2,4-dienoyl-CoA is converted to trans-2-enoyl-CoA by 2,4-dienoyl-CoA reductase and delta3-delta2-enoyl-CoA isomerase; trans-2-enoyl-CoA returns to the core beta-oxidation pathway for further degradation. Fatty acid beta-oxidation begins with the addition of coenzyme A to a fatty acid, and ends when only two or three carbons remain (as acetyl-CoA or propionyl-CoA respectively). Sources: GOC:mah, MetaCyc:PWY-5138